{
  "term_label": "Unknown cellular component",
  "term_id": "UNKNOWN:0003",
  "gene_symbol": "NDNF",
  "gene_name": "Protein NDNF",
  "gene": "UniProtKB:Q8TB73"
}